{
  "gene_symbol": "RPS6",
  "gene_name": "Small ribosomal subunit protein eS6",
  "term_label": "Unknown molecular function",
  "gene": "UniProtKB:P62753",
  "term_id": "UNKNOWN:0001"
}